{
  "gene": "UniProtKB:P01375",
  "term_id": "GO:0005125",
  "term_label": "cytokine activity",
  "gene_name": "Tumor necrosis factor",
  "gene_symbol": "TNF"
}